endopeptidase activity [GO:0004175] (molecular function) Definition: Catalysis of the hydrolysis of internal, alpha-peptide bonds in a polypeptide chain. Sources: http://merops.sanger.ac.uk/about/glossary.htm#ENDOPEPTIDASE Also known as: endoprotease activity, proteasome endopeptidase activity, proteinase, elastase activity Relationships: is a type of peptidase activity [GO:0008233] Subtypes: aspartic-type endopeptidase activity [GO:0004190], GO:0004197, metalloendopeptidase activity [GO:0004222], GO:0004252, GO:0004298, signal peptidase activity [GO:0009003], peptidoglycan endopeptidase activity [GO:0061785], glutamic-type endopeptidase activity [GO:0070007], oligopeptidase activity [GO:0070012] Regulation: negatively regulated by GO:0004866; positively regulated by GO:0010950; negatively regulated by negative regulation of endopeptidase activity [GO:0010951]; regulated by GO:0052548; positively regulated by endopeptidase activator activity [GO:0061133]; regulated by endopeptidase regulator activity [GO:0061135]